{
  "term_label": "Unknown molecular function",
  "gene_name": "NF-kappa-B inhibitor beta",
  "gene": "UniProtKB:Q15653",
  "term_id": "UNKNOWN:0001",
  "gene_symbol": "NFKBIB"
}